{
  "term_id": "GO:0005737",
  "gene_name": "Phospholipase A and acyltransferase 1",
  "gene_symbol": "PLAAT1",
  "gene": "UniProtKB:Q9HDD0",
  "term_label": "cytoplasm"
}